{
  "gene_name": "Terminal nucleotidyltransferase 5B",
  "gene": "UniProtKB:Q96A09",
  "term_id": "GO:1990817",
  "term_label": "poly(A) RNA polymerase activity",
  "gene_symbol": "TENT5B"
}